{
  "term_label": "cytoplasm",
  "term_id": "GO:0005737",
  "gene_name": "Protein pelota homolog",
  "gene_symbol": "PELO",
  "gene": "UniProtKB:Q9BRX2"
}